{
  "gene_name": "Psoriasis susceptibility 1 candidate gene 1 protein",
  "gene_symbol": "PSORS1C1",
  "term_id": "UNKNOWN:0001",
  "term_label": "Unknown molecular function",
  "gene": "UniProtKB:Q9UIG5"
}